negative regulation of transcription elongation by RNA polymerase I [GO:2001208] (biological process) Relationships: is a type of negative regulation of transcription by RNA polymerase I [GO:0016479]; is a type of negative regulation of DNA-templated transcription, elongation [GO:0032785]; is a type of GO:2001207; negatively regulates GO:0006362 Also known as: negative regulation of RNA elongation from Pol I promoter, negative regulation of transcription elongation from RNA polymerase I promoter Definition: Any process that stops, prevents or reduces the frequency, rate or extent of transcription elongation mediated by RNA polymerase I. References: PMID:20299458